inferior colliculus development [GO:0061379] (biological process) Relationships: is_a anatomical structure development [GO:0048856]; is part of corpora quadrigemina development [GO:0061378] Sources: GOC:dph, GOC:yaf Definition: The process whose specific outcome is the progression of the inferior colliculus over time, from its formation to the mature structure. The inferior colliculus (IC) (Latin, lower hill) is the principal midbrain nucleus of the auditory pathway and receives input from several more peripheral brainstem nuclei in the auditory pathway, as well as inputs from the auditory cortex. The inferior colliculus has three subdivisions: the central nucleus (CIC), a dorsal cortex (DCIC) by which it is surrounded, and an external cortex (ICX) which is located laterally.